{
  "gene_name": "Tubulin alpha 3f pseudogene",
  "gene_symbol": "TUBA3FP",
  "gene": "UniProtKB:A0A994J5G1",
  "term_label": "Unknown biological process",
  "term_id": "UNKNOWN:0002"
}